{
  "term_id": "GO:0071933",
  "term_label": "Arp2/3 complex binding",
  "gene_name": "Glia maturation factor beta",
  "gene": "UniProtKB:P60983",
  "gene_symbol": "GMFB"
}